{
  "gene_name": "Olfactory receptor 5P2",
  "term_id": "UNKNOWN:0003",
  "gene": "UniProtKB:Q8WZ92",
  "gene_symbol": "OR5P2",
  "term_label": "Unknown cellular component"
}